{
  "gene_name": "Harmonin",
  "term_id": "GO:0005929",
  "gene_symbol": "USH1C",
  "term_label": "cilium",
  "gene": "UniProtKB:Q9Y6N9"
}